sulfite transmembrane transporter activity [GO:0000319] (molecular function) Definition: Enables the transfer of sulfite ions from one side of a membrane to the other. Also known as: sulphite transporter activity Relationships: is a type of GO:1901682; is part of sulfite transmembrane transport [GO:0000316] Sources: GOC:as